{
  "gene": "UniProtKB:Q6UB98",
  "term_id": "GO:0005654",
  "gene_symbol": "ANKRD12",
  "term_label": "nucleoplasm",
  "gene_name": "Ankyrin repeat domain-containing protein 12"
}